3-(2,3-dihydroxyphenyl)propanoate catabolic process [GO:1901791] (biological process) Definition: The chemical reactions and pathways resulting in the breakdown of 3-(2,3-dihydroxyphenyl)propanoate. Also known as: 3-(2,3-dihydroxyphenyl)propanoate breakdown, 3-(2,3-dihydroxyphenyl)propanoate catabolism, 3-(2,3-dihydroxyphenyl)propanoate degradation Sources: GOC:TermGenie, GOC:yaf, MetaCyc:HCAMHPDEG-PWY, UniPathway:UPA00836 Relationships: is_a catechol-containing compound catabolic process [GO:0019614]; is a type of monocarboxylic acid catabolic process [GO:0072329]